separase-securin complex [GO:1990520] (cellular component) Definition: A protein complex that includes separase (a protease which cleaves cohesin as part of chromosome separation) and securin, a protease inhibitor. Chromosome separation is inhibited until securin is degraded by the Anaphase Promoting Complex (APC). References: PMID:8978688 Sources: GOC:dos, GOC:vw Also known as: Cut1-2 complex Relationships: is a type of endopeptidase complex [GO:1905369]